sulfur carrier activity [GO:0097163] (molecular function) Relationships: is a type of molecular carrier activity [GO:0140104] References: PMID:16387657 Sources: GOC:imk Definition: Covalently binding to sulfur and delivering it to an acceptor molecule.